{
  "gene": "UniProtKB:Q8TAP8",
  "gene_symbol": "PPP1R35",
  "term_id": "GO:0005814",
  "gene_name": "Protein phosphatase 1 regulatory subunit 35",
  "term_label": "centriole"
}